positive regulation of DNA-binding transcription factor activity [GO:0051091] (biological process) Sources: GOC:ai Relationships: is a type of GO:0044093; is a type of regulation of DNA-binding transcription factor activity [GO:0051090]; RO_0002213 DNA-binding transcription factor activity [GO:0003700] Subtypes: GO:0032793, positive regulation of NF-kappaB transcription factor activity [GO:0051092], positive regulation of androgen receptor activity [GO:2000825] Also known as: positive regulation of transcription factor activity, positive regulation of DNA binding transcription factor activity, positive regulation of sequence-specific DNA binding transcription factor activity, up regulation of transcription factor activity, up-regulation of transcription factor activity, upregulation of transcription factor activity, activation of transcription factor activity, positive regulation of thyroid hormone receptor activity, stimulation of transcription factor activity Definition: Any process that activates or increases the frequency, rate or extent of activity of a transcription factor, any factor involved in the initiation or regulation of transcription.